{
  "gene_name": "E3 ubiquitin-protein ligase UBR2",
  "term_id": "GO:0005737",
  "term_label": "cytoplasm",
  "gene_symbol": "UBR2",
  "gene": "UniProtKB:Q8IWV8"
}